{
  "term_id": "GO:0061507",
  "gene": "UniProtKB:Q86WV6",
  "term_label": "2',3'-cyclic GMP-AMP binding",
  "gene_name": "Stimulator of interferon genes protein",
  "gene_symbol": "STING1"
}